{
  "term_label": "DNA-binding transcription factor activity, RNA polymerase II-specific",
  "gene_name": "Zinc finger protein 354B",
  "term_id": "GO:0000981",
  "gene_symbol": "ZNF354B",
  "gene": "UniProtKB:Q96LW1"
}